cholesterol transport involved in cholesterol storage [GO:0010879] (biological process) Definition: The directed movement of cholesterol into cells that is part of their accumulation and maintenance. Sources: GOC:dph, GOC:tb Relationships: is a type of lipid transport involved in lipid storage [GO:0010877]; is a type of GO:0030301; is part of GO:0010878